{
  "gene": "UniProtKB:Q969X2",
  "gene_name": "Alpha-N-acetylgalactosaminide alpha-2,6-sialyltransferase 6",
  "term_id": "GO:0001574",
  "term_label": "ganglioside biosynthetic process",
  "gene_symbol": "ST6GALNAC6"
}